{
  "gene_name": "Polypeptide N-acetylgalactosaminyltransferase 9",
  "gene_symbol": "GALNT9",
  "term_id": "GO:0004653",
  "gene": "UniProtKB:Q9HCQ5",
  "term_label": "polypeptide N-acetylgalactosaminyltransferase activity"
}